{
  "gene_name": "Peroxisomal ATPase PEX6",
  "gene_symbol": "PEX6",
  "gene": "UniProtKB:Q13608",
  "term_label": "peroxisomal membrane",
  "term_id": "GO:0005778"
}